aliphatic (S)-hydroxynitrile lyase activity [GO:0052891] (molecular function) References: PMID:15299689 Definition: Catalysis of the reaction: an aliphatic (S)-hydroxynitrile = an aliphatic aldehyde or ketone + cyanide. Also known as: (S)-cyanohydrin carbonyl-lyase (cyanide forming) activity, (S)-cyanohydrin producing hydroxynitrile lyase activity, (S)-hydroxynitrile lyase activity, (S)-oxynitrilase activity, (S)-selective hydroxynitrile lyase activity Relationships: is a type of GO:0047606